{
  "gene_symbol": "ZNF84",
  "gene_name": "Zinc finger protein 84",
  "term_id": "UNKNOWN:0001",
  "term_label": "Unknown molecular function",
  "gene": "UniProtKB:P51523"
}